CBF3 complex [GO:0031518] (cellular component) References: PMID:13679521, PMID:9407032 Relationships: is a type of nuclear protein-containing complex [GO:0140513]; BFO_0000050 chromosome, centromeric region [GO:0000775] Definition: A multisubunit protein complex that binds to centromeric DNA and initiates kinetochore assembly. In yeast, this complex consists of four subunits, namely Ctf13p, Skp1p, Cep3p and Cbf2p.